{
  "gene_symbol": "PRKD3",
  "term_id": "GO:0035556",
  "gene_name": "Serine_threonine-protein kinase D3",
  "term_label": "intracellular signal transduction",
  "gene": "UniProtKB:O94806"
}